delta1-pyrroline-5-carboxylate synthetase activity [GO:0017084] (molecular function) Also known as: D1-pyrroline-5-carboxylate synthetase activity Sources: RHEA:33207 Relationships: is a type of oxidoreductase activity, acting on the aldehyde or oxo group of donors, NAD or NADP as acceptor [GO:0016620] Definition: Catalysis of the reaction: ATP + H+ + L-glutamate + NADPH = ADP + L-glutamate 5-semialdehyde + NADP+ + phosphate.